type A cholecystokinin receptor binding [GO:0031740] (molecular function) Sources: GOC:mah, GOC:nln Definition: Binding to a type A cholecystokinin receptor. Also known as: type A cholecystokinin receptor ligand Relationships: is a type of GO:0031739